{
  "gene_name": "Cilia- and flagella-associated protein 69",
  "term_label": "olfactory behavior",
  "gene_symbol": "CFAP69",
  "gene": "UniProtKB:A5D8W1",
  "term_id": "GO:0042048"
}